contractile vacuole pore [GO:0031913] (cellular component) Definition: Stable structure that regulates the flow of liquid between the contractile vacuole and the surrounding medium. Relationships: is a type of plasma membrane protein complex [GO:0098797]; is part of cytoskeleton [GO:0005856]; is part of contractile vacuolar membrane [GO:0031164] References: PMID:10503189